{
  "term_id": "GO:0006629",
  "term_label": "lipid metabolic process",
  "gene_name": "Acyl-CoA wax alcohol acyltransferase 1",
  "gene": "UniProtKB:Q58HT5",
  "gene_symbol": "AWAT1"
}